{
  "gene_symbol": "CHCHD2P9",
  "gene_name": "Putative coiled-coil-helix-coiled-coil-helix domain-containing protein CHCHD2P9, mitochondrial",
  "term_label": "mitochondrion",
  "term_id": "GO:0005739",
  "gene": "UniProtKB:Q5T1J5"
}